{
  "term_label": "positive regulation of proteasomal ubiquitin-dependent protein catabolic process",
  "gene": "UniProtKB:Q9BW61",
  "gene_name": "DET1- and DDB1-associated protein 1",
  "gene_symbol": "DDA1",
  "term_id": "GO:0032436"
}